{
  "gene": "UniProtKB:Q5T7N2",
  "gene_symbol": "L1TD1",
  "gene_name": "LINE-1 type transposase domain-containing protein 1",
  "term_label": "retrotransposition",
  "term_id": "GO:0032197"
}